purine nucleoside metabolic process [GO:0042278] (biological process) Sources: GOC:jl, ISBN:0140512713 Subtypes: GO:0006152, purine nucleoside interconversion [GO:0019686], purine nucleoside biosynthetic process [GO:0042451], purine deoxyribonucleoside metabolic process [GO:0046122], GO:0046128 Definition: The chemical reactions and pathways involving one of a family of organic molecules consisting of a purine base covalently bonded to a sugar ribose (a ribonucleoside) or deoxyribose (a deoxyribonucleoside). Also known as: purine metabolic process, purine metabolism, purine nucleoside metabolism Relationships: is a type of GO:0009116; is a type of purine-containing compound metabolic process [GO:0072521]